{
  "gene": "UniProtKB:Q9Y2D8",
  "term_id": "GO:0035735",
  "term_label": "intraciliary transport involved in cilium assembly",
  "gene_name": "Afadin- and alpha-actinin-binding protein",
  "gene_symbol": "SSX2IP"
}